7-methylguanosine biosynthetic process [GO:0046118] (biological process) Relationships: is a type of 7-methylguanosine metabolic process [GO:0008618]; is a type of guanosine-containing compound biosynthetic process [GO:1901070] Definition: The chemical reactions and pathways resulting in the formation of 7-methylguanosine, a modified nucleoside that forms a cap at the 5'-terminus of eukaryotic mRNA. Sources: ISBN:0198506732 Also known as: 7-methylguanosine anabolism, 7-methylguanosine biosynthesis, 7-methylguanosine formation, 7-methylguanosine synthesis